{
  "gene": "UniProtKB:Q9NZC2",
  "term_label": "positive regulation of calcium-mediated signaling",
  "gene_symbol": "TREM2",
  "gene_name": "Triggering receptor expressed on myeloid cells 2",
  "term_id": "GO:0050850"
}